{
  "term_label": "1-phosphatidylinositol-4,5-bisphosphate 3-kinase activity",
  "term_id": "GO:0046934",
  "gene_name": "Phosphatidylinositol 4,5-bisphosphate 3-kinase catalytic subunit gamma isoform",
  "gene": "UniProtKB:P48736",
  "gene_symbol": "PIK3CG"
}